somatic embryogenesis [GO:0010262] (biological process) Relationships: is a type of embryo development ending in seed dormancy [GO:0009793]; is a type of regeneration [GO:0031099] Definition: Initiation of a somatic embryo-an embryo arising from previously differentiated somatic cells, rather than from fused haploid gametes. References: PMID:9611173 Sources: GOC:sm